{
  "term_id": "GO:0010506",
  "gene_symbol": "RPTOR",
  "gene": "UniProtKB:Q8N122",
  "term_label": "regulation of autophagy",
  "gene_name": "Regulatory-associated protein of mTOR"
}